{
  "term_label": "Unknown cellular component",
  "term_id": "UNKNOWN:0003",
  "gene_symbol": "LOC101059948",
  "gene": "UniProtKB:A0A1B0GTJ6",
  "gene_name": "HCG1796489"
}